{
  "gene_name": "Ribulose-phosphate 3-epimerase-like protein 1",
  "gene": "UniProtKB:Q2QD12",
  "gene_symbol": "RPEL1",
  "term_id": "GO:0009052",
  "term_label": "pentose-phosphate shunt, non-oxidative branch"
}